{
  "gene_name": "Olfactory receptor 4A8",
  "gene": "UniProtKB:P0C604",
  "gene_symbol": "OR4A8",
  "term_id": "GO:0004984",
  "term_label": "olfactory receptor activity"
}